{
  "term_label": "Unknown cellular component",
  "gene": "UniProtKB:Q11130",
  "term_id": "UNKNOWN:0003",
  "gene_name": "Alpha-(1,3)-fucosyltransferase 7",
  "gene_symbol": "FUT7"
}